{
  "gene_symbol": "SRRD",
  "gene_name": "SRR1-like protein",
  "term_id": "GO:0005737",
  "gene": "UniProtKB:Q9UH36",
  "term_label": "cytoplasm"
}